protein K48-linked deubiquitination [GO:0071108] (biological process) Sources: GOC:mah Relationships: is a type of protein deubiquitination [GO:0016579] Definition: A protein deubiquitination process in which a K48-linked ubiquitin chain, i.e. a polymer of ubiquitin formed by linkages between lysine residues at position 48 of the ubiquitin monomers, is removed from a protein. Regulation: regulated by GO:1903093; negatively regulated by negative regulation of protein K48-linked deubiquitination [GO:1903094]